regulation of interleukin-21 production [GO:0032665] (biological process) Subtypes: negative regulation of interleukin-21 production [GO:0032705], positive regulation of interleukin-21 production [GO:0032745] Definition: Any process that modulates the frequency, rate, or extent of interleukin-21 production. Relationships: is a type of regulation of cytokine production [GO:0001817]; regulates interleukin-21 production [GO:0032625] Sources: GOC:mah Also known as: regulation of IL-21 production, regulation of interleukin-21 biosynthetic process